regulation of male pigmentation [GO:0048088] (biological process) Sources: GOC:jid Relationships: is a type of GO:0048070; is a type of regulation of developmental process [GO:0050793]; is a type of regulation of reproductive process [GO:2000241]; regulates male pigmentation [GO:0048094] Subtypes: negative regulation of male pigmentation [GO:0048092], positive regulation of male pigmentation [GO:0048093] Definition: Any process that modulates the frequency, rate or extent of establishment of a pattern of pigment in males.